{
  "gene_name": "G-protein coupled receptor 52",
  "gene_symbol": "GPR52",
  "term_id": "GO:0071482",
  "term_label": "cellular response to light stimulus",
  "gene": "UniProtKB:Q9Y2T5"
}